arachidonate binding [GO:0050544] (molecular function) Definition: Binding to arachidonic acid, a straight chain fatty acid with 20 carbon atoms and four double bonds per molecule. Arachidonic acid is the all-Z-(5,8,11,14)-isomer. Also known as: arachidonic acid binding Relationships: is a type of icosanoid binding [GO:0050542]; is a type of GO:0050543 Sources: GOC:ai